{
  "term_id": "UNKNOWN:0002",
  "gene_symbol": "SYNPR",
  "term_label": "Unknown biological process",
  "gene": "UniProtKB:Q8TBG9",
  "gene_name": "Synaptoporin"
}